{
  "term_id": "UNKNOWN:0001",
  "gene_name": "Junctophilin-4",
  "gene_symbol": "JPH4",
  "term_label": "Unknown molecular function",
  "gene": "UniProtKB:Q96JJ6"
}